{
  "gene_name": "Coiled-coil domain-containing protein 120",
  "term_label": "Unknown biological process",
  "gene_symbol": "CCDC120",
  "gene": "UniProtKB:Q96HB5",
  "term_id": "UNKNOWN:0002"
}